{
  "gene_symbol": "EGFR",
  "gene": "UniProtKB:P00533",
  "term_id": "GO:0048408",
  "gene_name": "Epidermal growth factor receptor",
  "term_label": "epidermal growth factor binding"
}